para-aminobenzoyl-glutamate hydrolase activity [GO:0071713] (molecular function) References: PMID:20190044 Sources: GOC:imk Relationships: is a type of hydrolase activity, acting on carbon-nitrogen (but not peptide) bonds, in linear amides [GO:0016811] Definition: Catalysis of the reaction: para-aminobenzoyl-glutamate + H2O = para-aminobenzoate + L-glutamate.